{
  "term_label": "Unknown cellular component",
  "gene_symbol": "GFPT2",
  "term_id": "UNKNOWN:0003",
  "gene": "UniProtKB:O94808",
  "gene_name": "Glutamine--fructose-6-phosphate aminotransferase [isomerizing] 2"
}